{
  "gene": "UniProtKB:Q96NR3",
  "gene_name": "Patched domain-containing protein 1",
  "term_label": "chemical synaptic transmission",
  "term_id": "GO:0007268",
  "gene_symbol": "PTCHD1"
}